{
  "term_id": "GO:0004662",
  "term_label": "CAAX-protein geranylgeranyltransferase activity",
  "gene_symbol": "FNTA",
  "gene": "UniProtKB:P49354",
  "gene_name": "Protein farnesyltransferase_geranylgeranyltransferase type-1 subunit alpha"
}